{
  "gene_symbol": "TRIP12",
  "gene": "UniProtKB:Q14669",
  "gene_name": "E3 ubiquitin-protein ligase TRIP12",
  "term_label": "ubiquitin protein ligase activity",
  "term_id": "GO:0061630"
}